{
  "gene": "UniProtKB:Q14141",
  "gene_symbol": "SEPTIN6",
  "term_id": "GO:0061640",
  "gene_name": "Septin-6",
  "term_label": "cytoskeleton-dependent cytokinesis"
}